microtubule cytoskeleton organization involved in mitosis [GO:1902850] (BP) References: PMID:18799626 Sources: GOC:TermGenie, GO_REF:0000060 Also known as: microtubule cytoskeleton organisation involved in mitosis, microtubule dynamics involved in mitosis, microtubule cytoskeleton organization and biogenesis involved in mitosis Subtypes: mitotic spindle organization [GO:0007052], GO:0040001, microtubule bundle formation involved in mitotic spindle midzone assembly [GO:1903562], microtubule anchoring at mitotic spindle pole body [GO:1990810] Relationships: is a type of microtubule cytoskeleton organization [GO:0000226]; is a type of GO:1903047 Definition: Any microtubule cytoskeleton organization that is involved in mitosis.